L-glutamate oxidase activity [GO:0050025] (molecular function) Definition: Catalysis of the reaction: L-glutamate + O2 + H2O = 2-oxoglutarate + NH3 + H2O2. Sources: RHEA:20728 Also known as: L-glutamate:oxygen oxidoreductase (deaminating), L-glutamic acid oxidase activity, glutamate (acceptor) dehydrogenase activity, glutamate oxidase activity, glutamic acid oxidase activity, glutamic dehydrogenase (acceptor) Relationships: is a type of L-amino-acid oxidase activity [GO:0001716]